{
  "term_label": "microtubule minus-end binding",
  "gene_name": "Gamma-tubulin complex component 3",
  "gene_symbol": "TUBGCP3",
  "term_id": "GO:0051011",
  "gene": "UniProtKB:Q96CW5"
}